{
  "gene_name": "Nucleoplasmin-3",
  "gene": "UniProtKB:O75607",
  "term_id": "GO:0003682",
  "gene_symbol": "NPM3",
  "term_label": "chromatin binding"
}